petal formation [GO:0048451] (biological process) Relationships: is a type of floral organ formation [GO:0048449]; is part of GO:0048446 Definition: The process that gives rise to the petal. This process pertains to the initial formation of a structure from unspecified parts. Sources: GOC:jid